positive regulation of dermatome development [GO:0061184] (BP) Sources: GOC:BHF, GOC:dph Definition: Any process that increases the rate, frequency, or extent of the progression of the dermatome over time, from its initial formation to the mature structure. The dermatome is the portion of a somite that will form skin. Relationships: is a type of positive regulation of embryonic development [GO:0040019]; is a type of regulation of dermatome development [GO:0061183]; positively regulates dermatome development [GO:0061054]